negative regulation of regulation of vascular associated smooth muscle cell membrane depolarization [GO:1904198] (biological process) Definition: Any process that stops, prevents or reduces the frequency, rate or extent of regulation of vascular smooth muscle cell membrane depolarization. References: PMID:20826763 Sources: GOC:TermGenie, GO_REF:0000058 Also known as: down regulation of regulation of vascular smooth muscle cell membrane depolarization, down-regulation of regulation of vascular smooth muscle cell membrane depolarization, downregulation of regulation of vascular smooth muscle cell membrane depolarization, negative regulation of regulation of vascular smooth muscle cell membrane depolarization, inhibition of regulation of vascular smooth muscle cell membrane depolarization Relationships: is a type of negative regulation of membrane depolarization [GO:1904180]; RO_0002212 regulation of vascular associated smooth muscle cell membrane depolarization [GO:1990736]